dehydropipecolic acid reductase [GO:0062046] (molecular function) References: PMID:27758894, PMID:28330936 Definition: Catalysis of the reaction: dehydropipecolic acid + NAD(P)H + H+ = L-pipecolic acid + NAD(P)+. Relationships: is a type of GO:0016646